{
  "term_id": "GO:0000340",
  "gene_symbol": "EIF4E3",
  "gene_name": "Eukaryotic translation initiation factor 4E type 3",
  "term_label": "RNA 7-methylguanosine cap binding",
  "gene": "UniProtKB:Q8N5X7"
}